cellular response to arachidonate [GO:1904551] (biological process) Definition: Any process that results in a change in state or activity of a cell (in terms of movement, secretion, enzyme production, gene expression, etc.) as a result of an arachidonic acid stimulus. Relationships: is a type of cellular response to fatty acid [GO:0071398]; is a type of response to arachidonate [GO:1904550] References: PMID:16382163 Sources: GOC:TermGenie, GO_REF:0000071 Also known as: cellular response to arachidonic acid